oculomotor nerve structural organization [GO:0021624] (biological process) Sources: GOC:cls, GOC:dgh, GOC:dph, GOC:jid, GO_REF:0000021 Relationships: is a type of cranial nerve structural organization [GO:0021604]; BFO_0000050 GO:0021622 Also known as: oculomotor nerve structural organisation, CN III structural organization Definition: The process that contributes to the act of creating the structural organization of the oculomotor nerve. This process pertains to the physical shaping of a rudimentary structure. This motor nerve innervates all extraocular muscles except the superior oblique and the lateral rectus muscles. The superior division supplies the levator palpebrae superioris and superior rectus muscles. The inferior division supplies the medial rectus, inferior rectus and inferior oblique muscles. This nerve also innervates the striated muscles of the eyelid. Pupillary constriction and lens movement are mediated by this nerve for near vision. In the orbit the inferior division sends branches that enter the ciliary ganglion where they form functional contacts (synapses) with the ganglion cells. The ganglion cells send nerve fibers into the back of the eye where they travel to ultimately innervate the ciliary muscle and the constrictor pupillae muscle.